{
  "term_label": "nucleus",
  "gene": "UniProtKB:Q9Y6Q3",
  "gene_symbol": "ZFP37",
  "gene_name": "Zinc finger protein 37 homolog",
  "term_id": "GO:0005634"
}